{
  "gene_name": "Myosin-14",
  "gene_symbol": "MYH14",
  "gene": "UniProtKB:Q7Z406",
  "term_id": "GO:0016460",
  "term_label": "myosin II complex"
}